{
  "term_label": "Unknown biological process",
  "gene_symbol": "TRAJ24",
  "gene_name": "T cell receptor alpha joining 24 (Fragment)",
  "term_id": "UNKNOWN:0002",
  "gene": "UniProtKB:A0A075B6Z9"
}